cellular oxidant detoxification [GO:0098869] (biological process) Sources: GOC:dos, GOC:vw Subtypes: removal of superoxide radicals [GO:0019430], cellular detoxification of hydrogen peroxide [GO:0061692] Relationships: is a type of cellular detoxification [GO:1990748] Definition: Any process carried out at the cellular level that reduces or removes the toxicity superoxide radicals or hydrogen peroxide.